{
  "term_id": "GO:0005634",
  "gene_name": "Zinc finger protein 610",
  "gene": "UniProtKB:Q8N9Z0",
  "gene_symbol": "ZNF610",
  "term_label": "nucleus"
}